{
  "gene": "UniProtKB:Q00796",
  "gene_name": "Sorbitol dehydrogenase",
  "gene_symbol": "SORD",
  "term_id": "GO:0006062",
  "term_label": "sorbitol catabolic process"
}